{
  "gene": "UniProtKB:Q96BI3",
  "gene_symbol": "APH1A",
  "gene_name": "Gamma-secretase subunit APH-1A",
  "term_label": "Notch signaling pathway",
  "term_id": "GO:0007219"
}